{
  "gene": "UniProtKB:Q58FG0",
  "term_label": "Unknown molecular function",
  "gene_name": "Putative heat shock protein HSP 90-alpha A5",
  "term_id": "UNKNOWN:0001",
  "gene_symbol": "HSP90AA5P"
}